{
  "term_id": "UNKNOWN:0003",
  "gene": "UniProtKB:P0CG42",
  "gene_name": "Putative protein FAM157B",
  "term_label": "Unknown cellular component",
  "gene_symbol": "FAM157B"
}